{
  "gene_name": "Vasopressin V2 receptor",
  "gene_symbol": "AVPR2",
  "term_id": "GO:0005000",
  "gene": "UniProtKB:P30518",
  "term_label": "vasopressin receptor activity"
}